{
  "gene": "UniProtKB:Q8N3R9",
  "term_id": "GO:0005912",
  "gene_name": "Protein PALS1",
  "term_label": "adherens junction",
  "gene_symbol": "PALS1"
}